2-deoxystreptamine catabolic process [GO:1901743] (biological process) Also known as: 2-deoxystreptamine breakdown, 2-deoxystreptamine catabolism, 2-deoxystreptamine degradation Definition: The chemical reactions and pathways resulting in the breakdown of 2-deoxystreptamine. Relationships: is_a polyol catabolic process [GO:0046174]; is a type of 2-deoxystreptamine metabolic process [GO:1901742] Sources: GOC:TermGenie, GOC:yaf